{
  "term_id": "UNKNOWN:0001",
  "gene_symbol": "OS9",
  "gene_name": "Protein OS-9",
  "gene": "UniProtKB:Q13438",
  "term_label": "Unknown molecular function"
}